{
  "term_label": "axoneme",
  "gene": "UniProtKB:Q6IQ19",
  "gene_symbol": "CCSAP",
  "term_id": "GO:0005930",
  "gene_name": "Centriole, cilia and spindle-associated protein"
}